{
  "gene_symbol": "C10orf105",
  "term_id": "UNKNOWN:0002",
  "gene": "UniProtKB:Q8TEF2",
  "gene_name": "Uncharacterized protein C10orf105",
  "term_label": "Unknown biological process"
}